type VI protein secretion system complex [GO:0033104] (cellular component) References: PMID:16432199, PMID:16763151 Sources: GOC:mlg Also known as: T6SS complex Definition: A complex of proteins that permits the transfer of proteins into the extracellular milieu or directly into host cells via the type VI secretion system. Proteins secreted by this complex do not require an N-terminal signal sequence. Relationships: is a type of protein-containing complex [GO:0032991]